{
  "gene_symbol": "ANTXR1",
  "term_id": "GO:0005886",
  "term_label": "plasma membrane",
  "gene": "UniProtKB:Q9H6X2",
  "gene_name": "Anthrax toxin receptor 1"
}